{
  "gene_symbol": "STARD3NL",
  "gene_name": "STARD3 N-terminal-like protein",
  "gene": "UniProtKB:O95772",
  "term_label": "late endosome membrane",
  "term_id": "GO:0031902"
}